symbiont-mediated suppression of host cholinergic synaptic transmission [GO:0044761] (biological process) Also known as: negative regulation by symbiont of host cholinergic synaptic transmission Relationships: is_a GO:0044759; is a type of symbiont-mediated perturbation of host cholinergic synaptic transmission [GO:0044760] References: PMID:37157163 Sources: GOC:jl Definition: A process in which a symbiont inhibits or disrupts the normal execution of cholinergic synaptic transmission, communication from a neuron to a target (neuron, muscle, or secretory cell) across a synapse via the neurotransmitter choline, in its host organism.